protein localization to astral microtubule [GO:1902888] (biological process) Definition: A process in which a protein is transported to, or maintained in, a location within an astral microtubule. Also known as: protein localisation in astral microtubule, protein localisation to astral microtubule, protein localization in astral microtubule Relationships: is_a GO:1902889; is a type of protein localization to cytoplasmic microtubule [GO:1905755] References: PMID:16054030 Sources: GOC:TermGenie, GOC:kmv, GO_REF:0000087